L-histidine transmembrane transport [GO:0089709] (biological process) Subtypes: L-histidine transmembrane export from vacuole [GO:0089708], L-histidine transmembrane import into vacuole [GO:0090513], GO:1903810, L-histidine transmembrane transport from lysosomal lumen to cytosol [GO:1904918] References: PMID:21307582 Definition: The directed movement of L-histidine across a membrane. Relationships: is a type of GO:0015695; is a type of GO:0015801; is a type of azole transmembrane transport [GO:0045117]; is a type of GO:1902475